iron chaperone activity [GO:0034986] (molecular function) Relationships: is a type of metallochaperone activity [GO:0016530]; has part iron ion binding [GO:0005506] Sources: GOC:BHF, GOC:vk Definition: Directly binding to and delivering iron ions to a target protein. Also known as: iron carrier activity